{
  "gene_name": "Olfactory receptor 52P1",
  "term_id": "GO:0005886",
  "gene": "UniProtKB:Q8NH57",
  "term_label": "plasma membrane",
  "gene_symbol": "OR52P1"
}